{
  "gene_symbol": "ARSH",
  "term_label": "Unknown cellular component",
  "term_id": "UNKNOWN:0003",
  "gene": "UniProtKB:Q5FYA8",
  "gene_name": "Arylsulfatase H"
}